heart trabecula morphogenesis [GO:0061384] (biological process) Definition: The process of shaping a trabecula in the heart. A trabecula is a small, often microscopic, tissue element in the form of a small beam, strut or rod, which generally has a mechanical function. Trabecula are usually but not necessarily, composed of dense collagenous tissue. Sources: GOC:dph Relationships: is a type of trabecula morphogenesis [GO:0061383] Subtypes: GO:0003222